{
  "gene": "UniProtKB:P61587",
  "gene_symbol": "RND3",
  "term_id": "GO:0005829",
  "term_label": "cytosol",
  "gene_name": "Rho-related GTP-binding protein RhoE"
}